{
  "gene_name": "Phospholipid transfer protein",
  "term_id": "GO:0034375",
  "gene_symbol": "PLTP",
  "gene": "UniProtKB:P55058",
  "term_label": "high-density lipoprotein particle remodeling"
}